negative regulation of mesenchymal cell proliferation involved in lung development [GO:2000791] (biological process) Definition: Any process that stops, prevents or reduces the frequency, rate or extent of mesenchymal cell proliferation involved in lung development. References: PMID:21513708 Relationships: is a type of negative regulation of developmental process [GO:0051093]; is_a GO:0051241; is a type of negative regulation of mesenchymal cell proliferation [GO:0072201]; is a type of regulation of mesenchymal cell proliferation involved in lung development [GO:2000790]; negatively regulates mesenchymal cell proliferation involved in lung development [GO:0060916]